histone H3K9 deacetylase activity, NAD-dependent [GO:0046969] (molecular function) Definition: Catalysis of the reaction: histone H3 N6-acetyl-L-lysine (position 9) + NAD+ + H2O = histone H3 L-lysine (position 9) + 2''-O-acetyl-ADP-D-ribose + nicotinamide. This reaction transfers an acetyl group attached to a lysine residue in H3K9 to NAD, producing nicotinamide. References: PMID:28450737 Note: Comment: Note that the residue position corresponds to the canonical human H3 histone (UniProtKB:P84243); this residue is conserved across all eukaryotes. Residue 1 is the first residue following removal of the initiating Methionine (Met). Note that each histone is encoded by multiple genes, and sequences may vary across different genes within an organism. Also known as: NAD-dependent H3-K9 histone deacetylase activity, NAD-dependent histone H3K9 deacetylase activity, NAD-dependent histone deacetylase activity (H3-K9 specific) Relationships: is a type of histone deacetylase activity, NAD-dependent [GO:0017136]; is_a histone H3K deacetylase activity [GO:0141050]